{
  "gene_symbol": "CD200R1L",
  "gene": "UniProtKB:Q6Q8B3",
  "term_label": "Unknown biological process",
  "gene_name": "Cell surface glycoprotein CD200 receptor 2",
  "term_id": "UNKNOWN:0002"
}